{
  "gene_symbol": "MAP2K1",
  "term_label": "neuron differentiation",
  "term_id": "GO:0030182",
  "gene_name": "Dual specificity mitogen-activated protein kinase kinase 1",
  "gene": "UniProtKB:Q02750"
}